{
  "term_id": "GO:0004373",
  "gene": "UniProtKB:P13807",
  "term_label": "alpha-1,4-glucan glucosyltransferase (UDP-glucose donor) activity",
  "gene_name": "Glycogen [starch] synthase, muscle",
  "gene_symbol": "GYS1"
}